{
  "term_label": "Unknown biological process",
  "gene": "UniProtKB:Q8N3G9",
  "gene_name": "Transmembrane protein 130",
  "gene_symbol": "TMEM130",
  "term_id": "UNKNOWN:0002"
}